{
  "gene": "UniProtKB:P51522",
  "term_id": "GO:0006357",
  "term_label": "regulation of transcription by RNA polymerase II",
  "gene_symbol": "ZNF83",
  "gene_name": "Zinc finger protein 83"
}